{
  "gene_symbol": "CACNA1C",
  "term_label": "voltage-gated calcium channel complex",
  "gene": "UniProtKB:Q13936",
  "gene_name": "Voltage-dependent L-type calcium channel subunit alpha-1C",
  "term_id": "GO:0005891"
}